{
  "gene_symbol": "MOK",
  "term_id": "GO:0005634",
  "term_label": "nucleus",
  "gene_name": "MAPK_MAK_MRK overlapping kinase",
  "gene": "UniProtKB:Q9UQ07"
}